{
  "gene": "UniProtKB:Q96T76",
  "gene_name": "MMS19 nucleotide excision repair protein homolog",
  "term_id": "GO:0051604",
  "gene_symbol": "MMS19",
  "term_label": "protein maturation"
}